{
  "term_label": "Unknown molecular function",
  "gene_name": "Protein CIP2A",
  "gene_symbol": "CIP2A",
  "gene": "UniProtKB:Q8TCG1",
  "term_id": "UNKNOWN:0001"
}